{
  "term_id": "GO:0060070",
  "gene": "UniProtKB:P36402",
  "gene_symbol": "TCF7",
  "gene_name": "Transcription factor 7",
  "term_label": "canonical Wnt signaling pathway"
}